{
  "term_label": "calcium ion binding",
  "gene_symbol": "DSC1",
  "gene_name": "Desmocollin-1",
  "term_id": "GO:0005509",
  "gene": "UniProtKB:Q08554"
}